response to hydrogen peroxide [GO:0042542] (biological process) Relationships: is a type of response to reactive oxygen species [GO:0000302] Subtypes: cellular response to hydrogen peroxide [GO:0070301] Sources: GOC:jl Definition: Any process that results in a change in state or activity of a cell or an organism (in terms of movement, secretion, enzyme production, gene expression, etc.) as a result of a hydrogen peroxide (H2O2) stimulus.